{
  "gene": "UniProtKB:Q9ULS5",
  "gene_symbol": "TMCC3",
  "gene_name": "Transmembrane and coiled-coil domain protein 3",
  "term_label": "Unknown biological process",
  "term_id": "UNKNOWN:0002"
}